{
  "gene": "UniProtKB:P19971",
  "gene_name": "Thymidine phosphorylase",
  "gene_symbol": "TYMP",
  "term_id": "UNKNOWN:0002",
  "term_label": "Unknown biological process"
}